positive regulation of cell proliferation involved in heart morphogenesis [GO:2000138] (biological process) Definition: Any process that activates or increases the frequency, rate or extent of cell proliferation involved in heart morphogenesis. Sources: GOC:dph Relationships: is a type of positive regulation of cell population proliferation [GO:0008284]; is a type of regulation of cell proliferation involved in heart morphogenesis [GO:2000136]; positively regulates cell proliferation involved in heart morphogenesis [GO:0061323] Subtypes: positive regulation of cell proliferation involved in heart valve morphogenesis [GO:0003251], positive regulation of cell proliferation involved in outflow tract morphogenesis [GO:1901964], positive regulation of cardioblast proliferation [GO:1905062]